{
  "gene": "UniProtKB:Q92502",
  "gene_symbol": "STARD8",
  "term_id": "GO:0005096",
  "gene_name": "StAR-related lipid transfer protein 8",
  "term_label": "GTPase activator activity"
}